{
  "gene_name": "T cell receptor beta variable 6-4",
  "gene_symbol": "TRBV6-4",
  "term_id": "UNKNOWN:0001",
  "term_label": "Unknown molecular function",
  "gene": "UniProtKB:A0A1B0GX49"
}